{
  "gene_name": "Synaptotagmin-9",
  "gene": "UniProtKB:Q86SS6",
  "term_label": "vesicle-mediated transport",
  "term_id": "GO:0016192",
  "gene_symbol": "SYT9"
}